{
  "gene_name": "Bone sialoprotein 2",
  "term_label": "Unknown cellular component",
  "gene_symbol": "IBSP",
  "gene": "UniProtKB:P21815",
  "term_id": "UNKNOWN:0003"
}